sodium:phosphate symporter activity [GO:0005436] (molecular function) Definition: Enables the transfer of a solute or solutes from one side of a membrane to the other according to the reaction: Na+(out) + phosphate(out) = Na+(in) + phosphate(in). Also known as: sodium/phosphate symporter activity, sodium-dependent phosphate transmembrane transporter activity Subtypes: high-affinity phosphate:sodium symporter activity [GO:0005316] Relationships: is a type of GO:0005315; is a type of solute:sodium symporter activity [GO:0015370] Sources: TC:2.A.1.14.6